{
  "gene_symbol": "XPO4",
  "gene": "UniProtKB:Q9C0E2",
  "term_id": "GO:0005643",
  "term_label": "nuclear pore",
  "gene_name": "Exportin-4"
}